{
  "gene": "UniProtKB:P0DOY5",
  "term_label": "Unknown cellular component",
  "gene_symbol": "IGHD1-1",
  "term_id": "UNKNOWN:0003",
  "gene_name": "Immunoglobulin heavy diversity 1-1"
}